{
  "gene_symbol": "STC1",
  "gene_name": "Stanniocalcin-1",
  "term_label": "extracellular space",
  "gene": "UniProtKB:P52823",
  "term_id": "GO:0005615"
}